{
  "term_label": "cilium movement involved in cell motility",
  "term_id": "GO:0060294",
  "gene": "UniProtKB:Q9NYC9",
  "gene_name": "Dynein axonemal heavy chain 9",
  "gene_symbol": "DNAH9"
}